{
  "gene_name": "Ankyrin repeat and SOCS box protein 7",
  "term_id": "UNKNOWN:0001",
  "gene_symbol": "ASB7",
  "term_label": "Unknown molecular function",
  "gene": "UniProtKB:Q9H672"
}